{
  "term_id": "UNKNOWN:0001",
  "gene_name": "26S proteasome non-ATPase regulatory subunit 2",
  "term_label": "Unknown molecular function",
  "gene": "UniProtKB:Q13200",
  "gene_symbol": "PSMD2"
}